{
  "gene": "UniProtKB:A8MYJ7",
  "gene_symbol": "TTC34",
  "term_id": "UNKNOWN:0002",
  "gene_name": "Tetratricopeptide repeat protein 34",
  "term_label": "Unknown biological process"
}